{
  "gene": "UniProtKB:Q8N1K5",
  "gene_symbol": "THEMIS",
  "gene_name": "Protein THEMIS",
  "term_label": "T cell receptor signaling pathway",
  "term_id": "GO:0050852"
}